{
  "gene_name": "H(+)_Cl(-) exchange transporter 3",
  "term_label": "voltage-gated chloride channel activity",
  "term_id": "GO:0005247",
  "gene_symbol": "CLCN3",
  "gene": "UniProtKB:P51790"
}